cholesterol-5,6-oxide hydrolase activity [GO:0033963] (molecular function) Also known as: 5,6alpha-epoxy-5alpha-cholestan-3beta-ol hydrolase activity, ChEH, cholesterol-epoxide hydrolase activity Definition: Catalysis of the reactions: 5,6alpha-epoxy-5alpha-cholestan-3beta-ol + H2O = cholestane-3beta-5alpha,6beta-triol, and 5,6beta-epoxy-5beta-cholestan-3beta-ol + H2O = cholestane-3beta-5alpha,6beta-triol. Relationships: is a type of ether hydrolase activity [GO:0016803] Sources: EC:3.3.2.11